{
  "gene_symbol": "MAFB",
  "term_label": "RNA polymerase II cis-regulatory region sequence-specific DNA binding",
  "gene": "UniProtKB:Q9Y5Q3",
  "term_id": "GO:0000978",
  "gene_name": "Transcription factor MafB"
}